{
  "term_id": "UNKNOWN:0003",
  "gene_name": "Transmembrane protein 182",
  "gene_symbol": "TMEM182",
  "term_label": "Unknown cellular component",
  "gene": "UniProtKB:Q6ZP80"
}